{
  "term_id": "GO:0005737",
  "term_label": "cytoplasm",
  "gene_name": "Bifunctional 3'-5' exonuclease_ATP-dependent helicase WRN",
  "gene": "UniProtKB:Q14191",
  "gene_symbol": "WRN"
}